branching involved in mammary gland duct morphogenesis [GO:0060444] (biological process) Subtypes: GO:0060655, mammary gland branching involved in thelarche [GO:0060744], mammary gland branching involved in pregnancy [GO:0060745] Regulation: regulated by regulation of branching involved in mammary gland duct morphogenesis [GO:0060762] Also known as: mammary gland branching morphogenesis Relationships: is a type of branching morphogenesis of an epithelial tube [GO:0048754]; is part of mammary gland duct morphogenesis [GO:0060603] Sources: GOC:dph Definition: The process in which the branching structure of the mammary gland duct is generated and organized. The mammary gland is a large compound sebaceous gland that in female mammals is modified to secrete milk.